negative regulation of conidiophore stalk development [GO:0070800] (biological process) Definition: Any process that stops, prevents, or reduces the frequency, rate or extent of conidiophore stalk development, a process that leads to the formation of a conidiophore stalk. The conidiophore stalk is part of a specialized hypha that extends aerially from the growth substrate and supports structures from which conidia, or asexual spores, develop. Sources: GOC:mah Relationships: is a type of negative regulation of developmental process [GO:0051093]; is a type of regulation of conidiophore stalk development [GO:0070799]; is a type of GO:2000242; negatively regulates GO:0070788